{
  "gene_name": "Sonic hedgehog protein",
  "gene": "UniProtKB:Q15465",
  "term_id": "GO:0005113",
  "term_label": "patched binding",
  "gene_symbol": "SHH"
}